vagus nerve development [GO:0021564] (biological process) Definition: The process whose specific outcome is the progression of the vagus nerve over time, from its formation to the mature structure. This nerve is primarily sensory but also has visceromotor components. It originates in the brain stem and controls many autonomic functions of the heart, lungs, stomach, pharynx, larynx, trachea, esophagus and other gastrointestinal tract components. It controls some motor functions such as speech. The sensory branches mediate sensation from the pharynx, larynx, thorax and abdomen; it also innervates taste buds in the epiglottis. Relationships: is a type of GO:0021545; is part of GO:0021783 Sources: GOC:cls, GOC:dgh, GOC:dph, GOC:jid, GO_REF:0000021 Also known as: cranial nerve X development, CN X development, cranial nerve 10 development